1-pyrroline-4-hydroxy-2-carboxylate deaminase activity [GO:0047425] (MF) Sources: EC:3.5.4.22, RHEA:10560 Relationships: is a type of hydrolase activity, acting on carbon-nitrogen (but not peptide) bonds, in cyclic amidines [GO:0016814]; is a type of GO:0019239 Also known as: 1-pyrroline-4-hydroxy-2-carboxylate aminohydrolase (decyclizing), HPC deaminase activity Definition: Catalysis of the reaction: 4-hydroxy-1-pyrroline-2-carboxylate + H2O + H+ = 2,5-dioxopentanoate + NH4.